{
  "term_id": "GO:0031106",
  "gene": "UniProtKB:Q9NQW6",
  "gene_name": "Anillin",
  "gene_symbol": "ANLN",
  "term_label": "septin ring organization"
}